{
  "gene": "UniProtKB:Q14934",
  "gene_name": "Nuclear factor of activated T-cells, cytoplasmic 4",
  "gene_symbol": "NFATC4",
  "term_id": "GO:0033173",
  "term_label": "calcineurin-NFAT signaling cascade"
}